pollen tube growth [GO:0009860] (biological process) Definition: Growth of pollen via tip extension of the intine wall. Sources: ISBN:0943088399 Regulation: regulated by regulation of pollen tube growth [GO:0080092] Relationships: is a type of developmental process involved in reproduction [GO:0003006]; is a type of cell tip growth [GO:0009932]; is a type of developmental cell growth [GO:0048588]; is part of GO:0048868